{
  "gene": "UniProtKB:P21730",
  "term_label": "phospholipase C-activating G protein-coupled receptor signaling pathway",
  "gene_symbol": "C5AR1",
  "term_id": "GO:0007200",
  "gene_name": "C5a anaphylatoxin chemotactic receptor 1"
}